{
  "gene": "UniProtKB:Q8WZA0",
  "term_id": "UNKNOWN:0002",
  "gene_name": "Protein LZIC",
  "gene_symbol": "LZIC",
  "term_label": "Unknown biological process"
}